{
  "gene_name": "Oxysterols receptor LXR-beta",
  "gene_symbol": "NR1H2",
  "gene": "UniProtKB:P55055",
  "term_label": "nuclear receptor activity",
  "term_id": "GO:0004879"
}